{
  "gene_symbol": "CUL1",
  "term_id": "GO:0031625",
  "gene_name": "Cullin-1",
  "term_label": "ubiquitin protein ligase binding",
  "gene": "UniProtKB:Q13616"
}